{
  "term_id": "GO:0005886",
  "term_label": "plasma membrane",
  "gene": "UniProtKB:Q8NGC5",
  "gene_symbol": "OR6J1",
  "gene_name": "Olfactory receptor 6J1"
}